{
  "gene_name": "N-acetylaspartate synthetase",
  "term_label": "L-aspartate N-acetyltransferase activity",
  "gene_symbol": "NAT8L",
  "gene": "UniProtKB:Q8N9F0",
  "term_id": "GO:0017188"
}